negative regulation of cardioblast proliferation [GO:1905061] (biological process) Definition: Any process that stops, prevents or reduces the frequency, rate or extent of cardioblast proliferation. References: PMID:24236097 Sources: GOC:BHF, GOC:BHF_miRNA, GOC:TermGenie, GOC:bc, GO_REF:0000058 Also known as: down regulation of cardioblast proliferation, down-regulation of cardioblast proliferation, downregulation of cardioblast proliferation, inhibition of cardioblast proliferation Relationships: is a type of regulation of cardioblast proliferation [GO:0003264]; is a type of GO:2000137; RO_0002212 cardioblast proliferation [GO:0003263]